{
  "gene_name": "Carboxy-terminal domain RNA polymerase II polypeptide A small phosphatase 2",
  "term_label": "Unknown cellular component",
  "gene": "UniProtKB:O14595",
  "gene_symbol": "CTDSP2",
  "term_id": "UNKNOWN:0003"
}